{
  "term_label": "N-acetylglucosamine metabolic process",
  "gene_symbol": "CHST6",
  "term_id": "GO:0006044",
  "gene": "UniProtKB:Q9GZX3",
  "gene_name": "Carbohydrate sulfotransferase 6"
}